{
  "term_label": "nucleus",
  "gene": "UniProtKB:Q9H2P0",
  "gene_name": "Activity-dependent neuroprotector homeobox protein",
  "gene_symbol": "ADNP",
  "term_id": "GO:0005634"
}